{
  "gene_name": "Lambda-crystallin homolog",
  "term_id": "GO:0050104",
  "gene": "UniProtKB:Q9Y2S2",
  "term_label": "L-gulonate 3-dehydrogenase activity",
  "gene_symbol": "CRYL1"
}